procollagen-proline 4-dioxygenase complex, alpha(II) type [GO:0070387] (cellular component) Definition: A procollagen-proline 4-dioxygenase complex that contains alpha subunits of the type II isoform; its activity is inhibited by poly(L-proline) only at high concentrations. Also known as: prolyl 4-hydroxylase complex (alpha(II)-type), procollagen-proline, 2-oxoglutarate-4-dioxygenase complex, alpha(II) type References: PMID:14500733, PMID:7753822 Relationships: is a type of procollagen-proline 4-dioxygenase complex [GO:0016222]